negative regulation of bicoid mRNA localization [GO:0045853] (biological process) Sources: GOC:go_curators Relationships: is a type of GO:0008359; is a type of GO:1904581; negatively regulates GO:0045450 Definition: Any process that stops, prevents, or reduces the frequency, rate or extent of the process in which bicoid mRNA is transported to, or maintained in, a specific location. Also known as: down regulation of bicoid mRNA localization, down-regulation of bicoid mRNA localization, downregulation of bicoid mRNA localization, negative regulation of bicoid mRNA localisation, inhibition of bicoid mRNA localization